{
  "term_label": "calcium-dependent protein binding",
  "gene": "UniProtKB:P04271",
  "gene_symbol": "S100B",
  "gene_name": "Protein S100-B",
  "term_id": "GO:0048306"
}